succinyl-CoA:(R)-benzylsuccinate CoA-transferase activity [GO:0033877] (molecular function) Relationships: is a type of GO:0008410 Also known as: succinyl-CoA:benzylsuccinate CoA-transferase activity, benzylsuccinate CoA-transferase activity, succinyl-CoA:(R)-2-benzylsuccinate CoA-transferase activity Sources: EC:2.8.3.15, RHEA:16469 Definition: Catalysis of the reaction: (R)-2-benzylsuccinate + succinyl-CoA = (R)-2-benzylsuccinyl-CoA + succinate.